{
  "term_id": "GO:0007165",
  "gene_name": "Immunoglobulin superfamily member 1",
  "term_label": "signal transduction",
  "gene": "UniProtKB:Q8N6C5",
  "gene_symbol": "IGSF1"
}